{
  "term_id": "GO:0003723",
  "gene_name": "RNA-binding protein 5",
  "gene_symbol": "RBM5",
  "gene": "UniProtKB:P52756",
  "term_label": "RNA binding"
}